{
  "term_label": "Unknown molecular function",
  "term_id": "UNKNOWN:0001",
  "gene_name": "Protein chibby homolog 2",
  "gene_symbol": "CBY2",
  "gene": "UniProtKB:Q8NA61"
}